{
  "term_label": "negative regulation of transcription by RNA polymerase II",
  "gene_symbol": "ZNF33A",
  "gene_name": "Zinc finger protein 33A",
  "term_id": "GO:0000122",
  "gene": "UniProtKB:Q06730"
}